{
  "gene_symbol": "SIK1",
  "gene": "UniProtKB:P57059",
  "term_label": "protein serine/threonine kinase activity",
  "term_id": "GO:0004674",
  "gene_name": "Serine_threonine-protein kinase SIK1"
}